{
  "term_id": "GO:0000977",
  "gene_symbol": "RBL1",
  "term_label": "RNA polymerase II transcription regulatory region sequence-specific DNA binding",
  "gene_name": "Retinoblastoma-like protein 1",
  "gene": "UniProtKB:P28749"
}